{
  "gene": "UniProtKB:Q58FF7",
  "term_label": "cellular response to heat",
  "term_id": "GO:0034605",
  "gene_name": "Putative heat shock protein HSP 90-beta-3",
  "gene_symbol": "HSP90AB3P"
}